{
  "gene_name": "Actin-like protein 7B",
  "term_label": "Unknown biological process",
  "gene": "UniProtKB:Q9Y614",
  "term_id": "UNKNOWN:0002",
  "gene_symbol": "ACTL7B"
}